regulation of ureter smooth muscle cell differentiation [GO:2000061] (biological process) Sources: GOC:mtg_kidney_jan10, GOC:obol, GOC:yaf Definition: Any process that modulates the frequency, rate or extent of ureter smooth muscle cell differentiation. Relationships: is a type of regulation of muscle organ development [GO:0048634]; is a type of regulation of smooth muscle cell differentiation [GO:0051150]; regulates ureter smooth muscle cell differentiation [GO:0072193] Subtypes: GO:2000062, GO:2000063